{
  "term_label": "cytoplasm",
  "term_id": "GO:0005737",
  "gene_symbol": "OTUD7B",
  "gene_name": "OTU domain-containing protein 7B",
  "gene": "UniProtKB:Q6GQQ9"
}